{
  "gene_symbol": "AGO4",
  "gene": "UniProtKB:Q9HCK5",
  "term_label": "single-stranded RNA binding",
  "term_id": "GO:0003727",
  "gene_name": "Protein argonaute-4"
}